{
  "gene_symbol": "PPP2R1A",
  "gene_name": "Serine_threonine-protein phosphatase 2A 65 kDa regulatory subunit A alpha isoform",
  "gene": "UniProtKB:P30153",
  "term_label": "protein phosphatase type 2A complex",
  "term_id": "GO:0000159"
}